trehalose catabolic process [GO:0005993] (biological process) Sources: GOC:jl, ISBN:0028623819 Definition: The chemical reactions and pathways resulting in the breakdown of trehalose, a disaccharide that consists of two molecules of glucose and is isomeric with sucrose. Relationships: is a type of trehalose metabolic process [GO:0005991]; is a type of GO:0046352 Regulation: positively regulated by positive regulation of trehalose catabolic process [GO:1901319] Also known as: mycose catabolic process, mycose catabolism, mykose catabolic process, mykose catabolism, trehalose breakdown, trehalose catabolism, trehalose degradation